{
  "term_label": "cellular response to hormone stimulus",
  "gene_name": "Vasopressin V1a receptor",
  "gene": "UniProtKB:P37288",
  "term_id": "GO:0032870",
  "gene_symbol": "AVPR1A"
}